{
  "gene": "UniProtKB:Q96LA6",
  "gene_name": "Fc receptor-like protein 1",
  "gene_symbol": "FCRL1",
  "term_id": "GO:0004888",
  "term_label": "transmembrane signaling receptor activity"
}